co-transcriptional RNA 3'-end processing, cleavage and polyadenylation pathway [GO:0180012] (biological process) References: PMID:31499460 Also known as: cotranscriptional 3'-end processing of RNA polymerase II transcripts Definition: Any process involved in transcription termination-coupled 3' processing of RNA polymerase II RNA transcripts by 3' end cleavage and addition of a poly(A) tail. Relationships: is a type of GO:0031123 Subtypes: co-transcriptional mRNA 3'-end processing, cleavage and polyadenylation pathway [GO:0180010], co-transcriptional lncRNA 3' end processing, cleavage and polyadenylation pathway [GO:0180034]